{
  "term_id": "UNKNOWN:0003",
  "gene": "UniProtKB:O43175",
  "term_label": "Unknown cellular component",
  "gene_name": "D-3-phosphoglycerate dehydrogenase",
  "gene_symbol": "PHGDH"
}